{
  "gene_name": "Transmembrane protein C1orf162",
  "gene": "UniProtKB:Q8NEQ5",
  "term_label": "Unknown cellular component",
  "gene_symbol": "C1orf162",
  "term_id": "UNKNOWN:0003"
}